{
  "gene_name": "Transcription factor 7",
  "gene_symbol": "TCF7",
  "term_id": "GO:0000978",
  "term_label": "RNA polymerase II cis-regulatory region sequence-specific DNA binding",
  "gene": "UniProtKB:P36402"
}